{
  "term_id": "UNKNOWN:0001",
  "gene_name": "Glutamate-rich protein 6",
  "gene": "UniProtKB:Q7L0X2",
  "term_label": "Unknown molecular function",
  "gene_symbol": "ERICH6"
}